{
  "gene_name": "Acetylcholine receptor subunit beta",
  "gene": "UniProtKB:P11230",
  "term_label": "membrane depolarization",
  "term_id": "GO:0051899",
  "gene_symbol": "CHRNB1"
}